{
  "gene_name": "Opalin",
  "gene_symbol": "OPALIN",
  "term_id": "UNKNOWN:0001",
  "term_label": "Unknown molecular function",
  "gene": "UniProtKB:Q96PE5"
}